{
  "gene_symbol": "EIF3D",
  "term_label": "eukaryotic translation initiation factor 3 complex",
  "gene_name": "Eukaryotic translation initiation factor 3 subunit D",
  "gene": "UniProtKB:O15371",
  "term_id": "GO:0005852"
}